{
  "gene": "UniProtKB:Q96LR2",
  "gene_name": "Leucine rich adaptor protein 1",
  "gene_symbol": "LURAP1",
  "term_label": "positive regulation of cytokine production",
  "term_id": "GO:0001819"
}